{
  "term_id": "GO:0000976",
  "gene": "UniProtKB:Q8NB50",
  "gene_name": "Zinc finger protein 62 homolog",
  "gene_symbol": "ZFP62",
  "term_label": "transcription cis-regulatory region binding"
}